{
  "gene_symbol": "PGPEP1L",
  "gene_name": "Pyroglutamyl-peptidase 1-like protein",
  "term_id": "GO:0008233",
  "term_label": "peptidase activity",
  "gene": "UniProtKB:A6NFU8"
}